filamentous growth of a unicellular organism [GO:0044180] (biological process) Relationships: is a type of filamentous growth [GO:0030447] Definition: The process in which a unicellular organism grows in a threadlike, filamentous shape. Sources: GOC:mtg_cambridge_2009